{
  "term_id": "GO:0007420",
  "gene": "UniProtKB:Q9BYU1",
  "term_label": "brain development",
  "gene_symbol": "PBX4",
  "gene_name": "Pre-B-cell leukemia transcription factor 4"
}